{
  "gene_symbol": "SLC26A9",
  "gene_name": "Solute carrier family 26 member 9",
  "term_id": "GO:1902476",
  "gene": "UniProtKB:Q7LBE3",
  "term_label": "chloride transmembrane transport"
}